{
  "term_id": "GO:0005886",
  "gene_symbol": "DNM3",
  "gene": "UniProtKB:Q9UQ16",
  "gene_name": "Dynamin-3",
  "term_label": "plasma membrane"
}